{
  "term_label": "Unknown molecular function",
  "gene": "UniProtKB:P98182",
  "gene_symbol": "ZNF200",
  "term_id": "UNKNOWN:0001",
  "gene_name": "Zinc finger protein 200"
}